muscle cell migration [GO:0014812] (biological process) Sources: CL:0000187, GOC:mtg_muscle Definition: The orderly movement of a muscle cell from one site to another, often during the development of a multicellular organism. Subtypes: GO:0014909, muscle cell chemotaxis toward tendon cell [GO:0036061], GO:0051451, myotube cell migration [GO:0110122] Relationships: is a type of GO:0016477